{
  "term_id": "GO:0007283",
  "gene": "UniProtKB:Q05952",
  "term_label": "spermatogenesis",
  "gene_symbol": "TNP2",
  "gene_name": "Nuclear transition protein 2"
}